ecdysone biosynthetic process [GO:0006697] (biological process) Sources: ISBN:0198506732 Also known as: ecdysone anabolism, ecdysone biosynthesis, ecdysone formation, ecdysone synthesis Relationships: is a type of ecdysone metabolic process [GO:0008205]; is a type of sterol biosynthetic process [GO:0016126]; is a type of ecdysteroid biosynthetic process [GO:0045456]; is a type of secondary alcohol biosynthetic process [GO:1902653] Definition: The chemical reactions and pathways resulting in the formation of ecdysone, (22R)-2-beta,3-beta,14,22,25-pentahydroxycholest-7-en-6-one, an ecdysteroid found in insects.